cellular response to brain-derived neurotrophic factor stimulus [GO:1990416] (biological process) Relationships: is a type of cellular response to nerve growth factor stimulus [GO:1990090] References: PMID:21958434 Also known as: cellular response to BDNF stimulus Definition: A process that results in a change in state or activity of a cell (in terms of movement, secretion, enzyme production, gene expression, etc.) as a result of a brain-derived neurotrophic factor stimulus.